protein-DNA covalent cross-linking repair [GO:0106300] (biological process) Also known as: resolution of protein-DNA covalent cross-linking Definition: The removal of covalent cross-link between DNA and a protein. References: PMID:31921408 Relationships: is a type of DNA repair [GO:0006281]